{
  "gene_symbol": "ARRDC4",
  "term_label": "plasma membrane",
  "gene_name": "Arrestin domain-containing protein 4",
  "term_id": "GO:0005886",
  "gene": "UniProtKB:Q8NCT1"
}